regulation of platelet aggregation [GO:0090330] (biological process) Sources: GOC:dph, GOC:tb Definition: Any process that modulates the rate, frequency or extent of platelet aggregation. Platelet aggregation is the adhesion of one platelet to one or more other platelets via adhesion molecules. Relationships: is a type of GO:0010543; is a type of regulation of homotypic cell-cell adhesion [GO:0034110]; RO_0002211 platelet aggregation [GO:0070527] Subtypes: negative regulation of platelet aggregation [GO:0090331], positive regulation of platelet aggregation [GO:1901731]